{
  "gene": "UniProtKB:Q5MNV8",
  "gene_symbol": "FBXO47",
  "gene_name": "F-box only protein 47",
  "term_id": "UNKNOWN:0001",
  "term_label": "Unknown molecular function"
}